{
  "term_label": "regulation of integrin-mediated signaling pathway",
  "term_id": "GO:2001044",
  "gene_name": "CD177 antigen",
  "gene_symbol": "CD177",
  "gene": "UniProtKB:Q8N6Q3"
}